{
  "gene_name": "Intraflagellar transport protein 22 homolog",
  "gene_symbol": "IFT22",
  "term_id": "GO:0003924",
  "term_label": "GTPase activity",
  "gene": "UniProtKB:Q9H7X7"
}